{
  "term_id": "GO:0007267",
  "gene": "UniProtKB:Q8NFK1",
  "gene_symbol": "GJC3",
  "term_label": "cell-cell signaling",
  "gene_name": "Gap junction gamma-3 protein"
}